secondary thickening [GO:0080191] (BP) Definition: Lateral growth of a plant axis (shoot axis or root) that is an increase in thickness resulting from formation of tissue from a secondary thickening meristem. Sources: JSTOR:4354165, PO:0025004, PO:0025414 Note: Occurs in shoot axes in some monocotyledons such as Dracaena, and rarely in roots of monocotyledons. Distinct from primary thickening, because it is distant from and generally discontinuous with the apical meristem. Relationships: is a type of lateral growth [GO:0080190]